negative regulation of slow-twitch skeletal muscle fiber contraction [GO:0031450] (biological process) Sources: GOC:dph, GOC:ef, GOC:mah, GOC:mtg_muscle, GOC:tb Also known as: down regulation of slow-twitch skeletal muscle contraction, down-regulation of slow-twitch skeletal muscle contraction, downregulation of slow-twitch skeletal muscle contraction, negative regulation of slow-twitch skeletal muscle contraction, inhibition of slow-twitch skeletal muscle contraction Relationships: is a type of regulation of slow-twitch skeletal muscle fiber contraction [GO:0031449]; is a type of negative regulation of striated muscle contraction [GO:0045988]; negatively regulates slow-twitch skeletal muscle fiber contraction [GO:0031444] Definition: Any process that stops, prevents, or reduces the frequency, rate or extent of slow-twitch skeletal muscle contraction.